{
  "gene_name": "Neuron navigator 1",
  "term_id": "GO:0007399",
  "gene": "UniProtKB:Q8NEY1",
  "gene_symbol": "NAV1",
  "term_label": "nervous system development"
}